{
  "gene_name": "DNA (cytosine-5)-methyltransferase 3A",
  "term_id": "GO:0045892",
  "gene_symbol": "DNMT3A",
  "term_label": "negative regulation of DNA-templated transcription",
  "gene": "UniProtKB:Q9Y6K1"
}